incipient cellular bud site [GO:0000131] (CC) Relationships: is a type of GO:0030427 Sources: GOC:clt Definition: The portion of the budding yeast plasma membrane where a daughter cell will emerge. The yeast marks this spot with bud-site selection proteins before bud emergence occurs. Actin is polarized to this spot just prior to and during bud emergence.